protein destabilization [GO:0031648] (BP) Also known as: negative regulation of protein stability, protein destabilisation Sources: GOC:mah Relationships: is a type of regulation of protein stability [GO:0031647] Definition: Any process that decreases the stability of a protein, making it more vulnerable to degradative processes or aggregation.